negative regulation of sterol import [GO:2000910] (biological process) Definition: Any process that stops, prevents or reduces the frequency, rate or extent of sterol import. Sources: GOC:obol Also known as: negative regulation of sterol influx, negative regulation of sterol uptake Relationships: is a type of negative regulation of sterol transport [GO:0032372]; is a type of regulation of sterol import [GO:2000909]; RO_0002212 sterol import [GO:0035376]